{
  "term_label": "Unknown molecular function",
  "gene_symbol": "APLP2",
  "gene_name": "Amyloid beta precursor like protein 2",
  "term_id": "UNKNOWN:0001",
  "gene": "UniProtKB:Q06481"
}